{
  "term_label": "receptor complex",
  "gene_symbol": "EPHA2",
  "gene": "UniProtKB:P29317",
  "term_id": "GO:0043235",
  "gene_name": "Ephrin type-A receptor 2"
}